negative regulation of neuron maturation [GO:0014043] (biological process) Subtypes: negative regulation of neuron remodeling [GO:1904800] Sources: GOC:ef Relationships: is a type of GO:0014041; is a type of negative regulation of cell maturation [GO:1903430]; RO_0002212 neuron maturation [GO:0042551] Also known as: down regulation of neuron maturation, down-regulation of neuron maturation, downregulation of neuron maturation, inhibition of neuron maturation Definition: Any process that stops, prevents, or reduces the frequency, rate or extent of neuron maturation.